{
  "gene_name": "SCY1-like protein 2",
  "gene": "UniProtKB:Q6P3W7",
  "term_id": "UNKNOWN:0001",
  "gene_symbol": "SCYL2",
  "term_label": "Unknown molecular function"
}